symbiont-mediated perturbation of host tight cell-cell junction [GO:0098865] (biological process) Relationships: is a type of symbiont-mediated perturbation of host cell-cell junction [GO:0044067] Subtypes: symbiont-mediated stabilization of host tight cell-cell junction [GO:0098864] Also known as: disruption of host tight cell-cell junction, disruption by symbiont of host tight cell-cell junction, modification by symbiont of host bicellular tight junctions, symbiont-mediated disruption of host tight cell-cell junction Definition: The process in which an organism effects a change that impairs the structure or temporarily subverts the tight cell-cell junctions between cells of the host. Tight cell-cell junctions, a cell-cell junction that seals cells together in an epithelium in a way that prevents even small molecules from leaking from one side of the sheet to the other. References: PMID:24287273